{
  "gene": "UniProtKB:Q14695",
  "gene_symbol": "KIAA0087",
  "gene_name": "Uncharacterized protein KIAA0087",
  "term_label": "Unknown cellular component",
  "term_id": "UNKNOWN:0003"
}